{
  "term_id": "GO:0006955",
  "gene": "UniProtKB:O75594",
  "term_label": "immune response",
  "gene_symbol": "PGLYRP1",
  "gene_name": "Peptidoglycan recognition protein 1"
}